melanosome membrane [GO:0033162] (cellular component) Definition: The lipid bilayer surrounding a melanosome. Sources: GOC:mah Relationships: is_a pigment granule membrane [GO:0090741]; is part of GO:0042470; is part of chitosome [GO:0045009]